{
  "gene_symbol": "BAX",
  "term_label": "positive regulation of neuron apoptotic process",
  "gene_name": "Apoptosis regulator BAX",
  "term_id": "GO:0043525",
  "gene": "UniProtKB:Q07812"
}